{
  "term_label": "Unknown cellular component",
  "gene_symbol": "PDCD2L",
  "term_id": "UNKNOWN:0003",
  "gene": "UniProtKB:Q9BRP1",
  "gene_name": "Programmed cell death protein 2-like"
}